solid phase of basement membrane [GO:0140139] (cellular component) Relationships: is_a external encapsulating structure [GO:0030312]; is part of basement membrane [GO:0005604] References: PMID:33972551 Definition: The solid compartment of the basement membrane ECM, including a specific subset of basement membrane collagens and basement membrane glycoproteins like laminins or nidogens.